positive regulation of collateral sprouting [GO:0048672] (biological process) Also known as: up regulation of collateral sprouting, up-regulation of collateral sprouting, upregulation of collateral sprouting, activation of collateral sprouting, stimulation of collateral sprouting Subtypes: positive regulation of collateral sprouting of intact axon in response to injury [GO:0048684], positive regulation of collateral sprouting of injured axon [GO:0048694], positive regulation of collateral sprouting in absence of injury [GO:0048697] Definition: Any process that activates or increases the frequency, rate or extent of collateral sprouting. Sources: GOC:dgh, GOC:dph, GOC:jid, GOC:lm Relationships: is a type of positive regulation of cell growth [GO:0030307]; is a type of positive regulation of developmental growth [GO:0048639]; is a type of GO:0048670; is a type of positive regulation of axonogenesis [GO:0050772]; positively regulates GO:0048668